{
  "gene_symbol": "SCAF8",
  "gene": "UniProtKB:Q9UPN6",
  "term_id": "GO:0005849",
  "term_label": "mRNA cleavage factor complex",
  "gene_name": "SR-related and CTD-associated factor 8"
}